{
  "gene_symbol": "CATSPER4",
  "gene_name": "Cation channel sperm-associated protein 4",
  "term_label": "sperm capacitation",
  "term_id": "GO:0048240",
  "gene": "UniProtKB:Q7RTX7"
}